{
  "gene_symbol": "LPXN",
  "term_label": "podosome",
  "term_id": "GO:0002102",
  "gene": "UniProtKB:O60711",
  "gene_name": "Leupaxin"
}